{
  "gene": "UniProtKB:Q06418",
  "gene_name": "Tyrosine-protein kinase receptor TYRO3",
  "term_id": "GO:0007169",
  "gene_symbol": "TYRO3",
  "term_label": "cell surface receptor protein tyrosine kinase signaling pathway"
}